{
  "term_label": "protein serine/threonine kinase activity",
  "gene": "UniProtKB:Q15831",
  "gene_symbol": "STK11",
  "gene_name": "Serine_threonine-protein kinase STK11",
  "term_id": "GO:0004674"
}